{
  "gene_symbol": "CBR1",
  "gene": "UniProtKB:P16152",
  "gene_name": "Carbonyl reductase [NADPH] 1",
  "term_id": "UNKNOWN:0002",
  "term_label": "Unknown biological process"
}